{
  "term_id": "UNKNOWN:0002",
  "term_label": "Unknown biological process",
  "gene_symbol": "KTN1",
  "gene_name": "Kinectin",
  "gene": "UniProtKB:Q86UP2"
}